thiamine metabolic process [GO:0006772] (biological process) Relationships: is a type of primary alcohol metabolic process [GO:0034308]; is a type of thiamine-containing compound metabolic process [GO:0042723] Definition: The chemical reactions and pathways involving thiamine (vitamin B1), a water soluble vitamin present in fresh vegetables and meats, especially liver. Also known as: thiamin metabolic process, thiamin metabolism, thiamine metabolism, vitamin B1 metabolic process, vitamin B1 metabolism Subtypes: GO:0009228, GO:0009230 Sources: GOC:jl, ISBN:0198506732